{
  "term_id": "UNKNOWN:0003",
  "gene_name": "Hepatocyte nuclear factor 3-alpha",
  "term_label": "Unknown cellular component",
  "gene": "UniProtKB:P55317",
  "gene_symbol": "FOXA1"
}